selenate transport [GO:0080160] (biological process) Relationships: is a type of GO:0015698 Definition: The directed movement of selenate into, out of or within a cell, or between cells, by means of some agent such as a transporter or pore. References: PMID:18761637